{
  "gene_symbol": "STUM",
  "term_label": "Unknown cellular component",
  "gene": "UniProtKB:Q69YW2",
  "term_id": "UNKNOWN:0003",
  "gene_name": "Protein stum homolog"
}